{
  "gene_symbol": "CORO7",
  "gene_name": "Coronin-7",
  "gene": "UniProtKB:P57737",
  "term_label": "plasma membrane",
  "term_id": "GO:0005886"
}